{
  "gene_symbol": "CTH",
  "term_id": "GO:0005737",
  "gene_name": "Cystathionine gamma-lyase",
  "term_label": "cytoplasm",
  "gene": "UniProtKB:P32929"
}